{
  "gene_name": "Interleukin-17 receptor D",
  "term_label": "interleukin-17 receptor activity",
  "gene_symbol": "IL17RD",
  "term_id": "GO:0030368",
  "gene": "UniProtKB:Q8NFM7"
}